{
  "gene": "UniProtKB:Q8WVC6",
  "gene_symbol": "DCAKD",
  "gene_name": "Dephospho-CoA kinase domain-containing protein",
  "term_label": "Unknown cellular component",
  "term_id": "UNKNOWN:0003"
}